positive regulation of maltotetraose transport [GO:1900323] (biological process) Sources: GOC:TermGenie, GOC:mengo_curators Also known as: up regulation of maltotetraose transport, up-regulation of maltotetraose transport, upregulation of maltotetraose transport, activation of maltotetraose transport Definition: Any process that activates or increases the frequency, rate or extent of maltotetraose transport. Relationships: is a type of positive regulation of transport [GO:0051050]; is a type of regulation of maltotetraose transport [GO:1900321]; positively regulates GO:2001099